{
  "term_id": "GO:0004252",
  "gene": "UniProtKB:Q9BZD6",
  "term_label": "serine-type endopeptidase activity",
  "gene_symbol": "PRRG4",
  "gene_name": "Transmembrane gamma-carboxyglutamic acid protein 4"
}